{
  "gene_symbol": "CXCR6",
  "gene": "UniProtKB:O00574",
  "gene_name": "C-X-C chemokine receptor type 6",
  "term_label": "immune response",
  "term_id": "GO:0006955"
}